{
  "term_label": "histone H3K14 deacetylase activity, NAD-dependent",
  "term_id": "GO:0032041",
  "gene_symbol": "SIRT1",
  "gene_name": "NAD-dependent protein deacetylase sirtuin-1",
  "gene": "UniProtKB:Q96EB6"
}